{
  "term_label": "Unknown cellular component",
  "term_id": "UNKNOWN:0003",
  "gene_symbol": "POLQ",
  "gene_name": "DNA polymerase theta",
  "gene": "UniProtKB:O75417"
}